luteolin-7-O-glucuronide 7-O-glucuronosyltransferase activity [GO:0047246] (molecular function) Relationships: is a type of GO:0015020 Also known as: LMT activity, UDP-glucuronate:luteolin 7-O-glucuronide-glucuronosyltransferase activity, UDP-glucuronate:luteolin-7-O-beta-D-glucuronide 2''-O-glucuronosyltransferase activity, luteolin-7-O-glucuronide 2''-O-glucuronosyltransferase activity, uridine diphosphoglucuronate-luteolin 7-O-glucuronide glucuronosyltransferase activity Sources: EC:2.4.1.190, RHEA:14149 Definition: Catalysis of the reaction: luteolin 7-O-beta-D-glucosiduronate + UDP-alpha-D-glucuronate = H+ + luteolin 7-O-[(beta-D-glucosiduronate)-(1->2)-(beta-D-glucosiduronate)] + UDP.